symbiont-mediated non-specific activation of host T-cells [GO:0141128] (BP) References: PMID:12679262, PMID:17427250, PMID:28880920 Also known as: symbiont-mediated non-specific T-cell activation in host, symbiont-mediated nonspecific activation of host T-cells Definition: A process by which a symbiont superantigen elicits a strong immune response by activating a large number of T cells in a non-specific manner. Unlike conventional antigens, which activate T cells by interacting with specific receptors on the surface of these cells, superantigens can stimulate T cells by binding to regions outside the antigen-binding site. Superantigens can activate a large proportion of T cells, leading to an exaggerated immune response. This excessive activation can result in the release of a large amount of cytokines such as tumor necrosis factor and interleukin-2. The massive cytokine release can lead to an acute toxic shock, causing symptoms such as fever and organ damage. Relationships: is a type of symbiont-mediated perturbation of host immune response [GO:0052553]